posterior cibarial plate morphogenesis [GO:0048720] (biological process) Definition: The process in which the anatomical structures of the posterior cibarial plate are generated and organized. Sources: GOC:rc Relationships: is a type of post-embryonic animal morphogenesis [GO:0009886]; is part of GO:0007453; is part of GO:0048727